{
  "term_id": "GO:0006325",
  "gene_symbol": "H2BC26",
  "gene": "UniProtKB:Q8N257",
  "term_label": "chromatin organization",
  "gene_name": "Histone H2B type 3-B"
}